{
  "term_id": "GO:0051015",
  "gene_symbol": "CTNNA3",
  "term_label": "actin filament binding",
  "gene_name": "Catenin alpha-3",
  "gene": "UniProtKB:Q9UI47"
}